{
  "term_label": "cell surface receptor protein tyrosine kinase signaling pathway",
  "gene_symbol": "STAP1",
  "gene": "UniProtKB:Q9ULZ2",
  "gene_name": "Signal-transducing adaptor protein 1",
  "term_id": "GO:0007169"
}